connexin binding [GO:0071253] (MF) References: PMID:19864490 Sources: GOC:mah Relationships: is a type of protein binding [GO:0005515] Definition: Binding to a connexin, any of a group of related proteins that assemble to form gap junctions.